{
  "gene_symbol": "MYO10",
  "term_label": "plus-end directed microfilament motor activity",
  "gene_name": "Unconventional myosin-X",
  "gene": "UniProtKB:Q9HD67",
  "term_id": "GO:0060002"
}